{
  "term_id": "GO:0005634",
  "gene_symbol": "ESCO1",
  "gene_name": "N-acetyltransferase ESCO1",
  "term_label": "nucleus",
  "gene": "UniProtKB:Q5FWF5"
}